{
  "gene": "UniProtKB:Q8TEH3",
  "gene_symbol": "DENND1A",
  "term_label": "clathrin-coated vesicle",
  "term_id": "GO:0030136",
  "gene_name": "DENN domain-containing protein 1A"
}